{
  "term_label": "Golgi apparatus",
  "gene": "UniProtKB:Q13445",
  "gene_name": "Transmembrane emp24 domain-containing protein 1",
  "gene_symbol": "TMED1",
  "term_id": "GO:0005794"
}